{
  "gene_symbol": "CREB5",
  "gene": "UniProtKB:Q02930",
  "term_id": "GO:0006357",
  "term_label": "regulation of transcription by RNA polymerase II",
  "gene_name": "Cyclic AMP-responsive element-binding protein 5"
}